{
  "gene_symbol": "SETD9",
  "term_id": "UNKNOWN:0003",
  "term_label": "Unknown cellular component",
  "gene": "UniProtKB:Q8NE22",
  "gene_name": "SET domain-containing protein 9"
}